{
  "gene_symbol": "TTC9",
  "gene_name": "Tetratricopeptide repeat protein 9A",
  "term_id": "UNKNOWN:0001",
  "gene": "UniProtKB:Q92623",
  "term_label": "Unknown molecular function"
}